{
  "gene_symbol": "CSNK2A1",
  "gene": "UniProtKB:P68400",
  "gene_name": "Casein kinase II subunit alpha",
  "term_id": "GO:0004674",
  "term_label": "protein serine/threonine kinase activity"
}